negative regulation of isopentenyl diphosphate biosynthetic process, methylerythritol 4-phosphate pathway [GO:0010323] (biological process) Also known as: down regulation of isopentenyl diphosphate biosynthetic process, mevalonate-independent pathway, down-regulation of isopentenyl diphosphate biosynthetic process, mevalonate-independent pathway, downregulation of isopentenyl diphosphate biosynthetic process, mevalonate-independent pathway, negative regulation of isopentenyl diphosphate biosynthetic process, mevalonate-independent pathway, inhibition of isopentenyl diphosphate biosynthetic process, mevalonate-independent pathway References: PMID:16531478 Definition: Any process that stops, prevents, or reduces the frequency, rate or extent of the chemical reactions and pathways resulting in the formation of isopentenyl diphosphate produced via the methylerythritol (MEP) pathway (mevalonate-independent). Relationships: is a type of regulation of isopentenyl diphosphate biosynthetic process, methylerythritol 4-phosphate pathway [GO:0010322]; is a type of negative regulation of isoprenoid metabolic process [GO:0045827]; is a type of negative regulation of carbohydrate metabolic process [GO:0045912]; is a type of negative regulation of phospholipid biosynthetic process [GO:0071072]; RO_0002212 isopentenyl diphosphate biosynthetic process, methylerythritol 4-phosphate pathway [GO:0019288]